GDP-fucose transmembrane transporter activity [GO:0005457] (molecular function) Relationships: is a type of purine nucleotide-sugar transmembrane transporter activity [GO:0036080]; is part of GO:0015783 Sources: GOC:ai, GOC:mtg_transport, ISBN:0815340729 Definition: Enables the transfer of a GDP-fucose from one side of a membrane to the other. GDP-fucose is a substance composed of fucose in glycosidic linkage with guanosine diphosphate.